positive regulation of circulating fibrinogen levels [GO:0061755] (biological process) Definition: Any process that increases the quantity of fibrinogen circulating in the bloodstream. Relationships: is a type of regulation of circulating fibrinogen levels [GO:0044537] References: PMID:20570858 Sources: GOC:BHF, GOC:BHF_miRNA, GOC:bf